mitochondrial membrane organization [GO:0007006] (biological process) Relationships: is a type of mitochondrion organization [GO:0007005]; is a type of membrane organization [GO:0061024]; occurs in mitochondrion [GO:0005739] Definition: A process that is carried out at the cellular level which results in the assembly, arrangement of constituent parts, or disassembly of a mitochondrial membrane, either of the lipid bilayer surrounding a mitochondrion. Sources: GOC:ai, GOC:dph, GOC:jl, GOC:mah Subtypes: inner mitochondrial membrane organization [GO:0007007], outer mitochondrial membrane organization [GO:0007008], GO:0046902, GO:0090151 Also known as: mitochondrial membrane organisation, mitochondrial membrane organization and biogenesis